{
  "term_label": "proteasome-mediated ubiquitin-dependent protein catabolic process",
  "gene_name": "PRAME family member 10",
  "term_id": "GO:0043161",
  "gene_symbol": "PRAMEF10",
  "gene": "UniProtKB:O60809"
}